{
  "gene": "UniProtKB:P55201",
  "gene_name": "Peregrin",
  "term_id": "GO:0005634",
  "term_label": "nucleus",
  "gene_symbol": "BRPF1"
}